pharyngeal system development [GO:0060037] (biological process) Sources: GOC:dph Definition: The process whose specific outcome is the progression of the pharyngeal system over time, from its formation to the mature structure. The pharyngeal system is a transient embryonic complex that is specific to vertebrates. It comprises the pharyngeal arches, bulges of tissues of mesoderm and neural crest derivation through which pass nerves and pharyngeal arch arteries. The arches are separated internally by pharyngeal pouches, evaginations of foregut endoderm, and externally by pharyngeal clefts, invaginations of surface ectoderm. The development of the system ends when the structure it contributes to are forming: the thymus, thyroid, parathyroids, maxilla, mandible, aortic arch, cardiac outflow tract, external and middle ear. Relationships: is a type of system development [GO:0048731]; is part of chordate embryonic development [GO:0043009]